{
  "term_id": "GO:0032991",
  "term_label": "protein-containing complex",
  "gene": "UniProtKB:Q8WXB1",
  "gene_name": "Protein N-lysine methyltransferase METTL21A",
  "gene_symbol": "METTL21A"
}